{
  "gene_name": "Tudor domain-containing protein 7",
  "term_id": "UNKNOWN:0001",
  "gene": "UniProtKB:Q8NHU6",
  "term_label": "Unknown molecular function",
  "gene_symbol": "TDRD7"
}